{
  "term_label": "mitotic spindle organization",
  "gene": "UniProtKB:O95239",
  "gene_name": "Chromosome-associated kinesin KIF4A",
  "term_id": "GO:0007052",
  "gene_symbol": "KIF4A"
}